C-terminal protein lipidation [GO:0006501] (biological process) Definition: The covalent attachment of a lipid group to the carboxy-terminus of a protein. Sources: GOC:jl Relationships: is a type of protein lipidation [GO:0006497]; is a type of C-terminal protein amino acid modification [GO:0018410] Subtypes: protein lipidation involved in autophagosome assembly [GO:0061739]